{
  "term_label": "nucleus",
  "gene": "UniProtKB:O75444",
  "gene_symbol": "MAF",
  "gene_name": "Transcription factor Maf",
  "term_id": "GO:0005634"
}